positive regulation of gamma-delta T cell activation involved in immune response [GO:2001193] (biological process) Definition: Any process that activates or increases the frequency, rate or extent of gamma-delta T cell activation involved in immune response. Sources: GOC:obol Also known as: positive regulation of gamma-delta T cell activation during immune response, positive regulation of gamma-delta T lymphocyte activation during immune response, positive regulation of gamma-delta T-cell activation during immune response, positive regulation of gamma-delta T-lymphocyte activation during immune response Relationships: is a type of positive regulation of immune effector process [GO:0002699]; is a type of positive regulation of gamma-delta T cell activation [GO:0046645]; is a type of GO:0050778; is a type of regulation of gamma-delta T cell activation involved in immune response [GO:2001191]; positively regulates gamma-delta T cell activation involved in immune response [GO:0002290]